{
  "term_id": "UNKNOWN:0001",
  "gene_symbol": "MARCHF6-DT",
  "gene_name": "Poly-ADP-ribosylation-amplifying and CtIP-maintaining micropeptide",
  "gene": "UniProtKB:P0DW81",
  "term_label": "Unknown molecular function"
}